ATP-dependent polyribonucleotide 5'-hydroxyl-kinase activity [GO:0051736] (molecular function) Sources: RHEA:54580 Relationships: is a type of GO:0051734 Also known as: polyribonucleotide 5'-hydroxyl-kinase activity, ATP-dependent RNA kinase activity, ATP-dependent polyribonucleotide kinase activity Definition: Catalysis of the reaction: ATP + 5'-dephospho-RNA = ADP + 5'-phospho-RNA.